{
  "gene_symbol": "ITGB1",
  "term_label": "C-X3-C chemokine binding",
  "gene": "UniProtKB:P05556",
  "term_id": "GO:0019960",
  "gene_name": "Integrin beta-1"
}